{
  "term_id": "GO:0050778",
  "gene_symbol": "HLA-DRA",
  "term_label": "positive regulation of immune response",
  "gene": "UniProtKB:P01903",
  "gene_name": "HLA class II histocompatibility antigen, DR alpha chain"
}